{
  "gene": "UniProtKB:Q99259",
  "gene_name": "Glutamate decarboxylase 1",
  "term_label": "cytoplasm",
  "term_id": "GO:0005737",
  "gene_symbol": "GAD1"
}